{
  "gene": "UniProtKB:Q5H8C1",
  "term_id": "GO:0031012",
  "gene_symbol": "FREM1",
  "gene_name": "FRAS1-related extracellular matrix protein 1",
  "term_label": "extracellular matrix"
}